{
  "gene": "UniProtKB:Q58FF6",
  "gene_name": "Putative heat shock protein HSP 90-beta 4",
  "term_label": "cellular response to heat",
  "term_id": "GO:0034605",
  "gene_symbol": "HSP90AB4P"
}